RNA polymerase II, core complex [GO:0005665] (cellular component) Definition: RNA polymerase II, one of three nuclear DNA-directed RNA polymerases found in all eukaryotes, is a multisubunit complex; typically it produces mRNAs, snoRNAs, and some of the snRNAs. Two large subunits comprise the most conserved portion including the catalytic site and share similarity with other eukaryotic and bacterial multisubunit RNA polymerases. The largest subunit of RNA polymerase II contains an essential carboxyl-terminal domain (CTD) composed of a variable number of heptapeptide repeats (YSPTSPS). The remainder of the complex is composed of smaller subunits (generally ten or more), some of which are also found in RNA polymerases I and III. Although the core is competent to mediate ribonucleic acid synthesis, it requires additional factors to select the appropriate template. Also known as: RNA polymerase II complex, RNAP II complex, DNA-directed RNA polymerase II, core complex Relationships: is a type of nuclear DNA-directed RNA polymerase complex [GO:0055029]; is part of RNA polymerase II, holoenzyme [GO:0016591] Sources: GOC:krc, GOC:mtg_sensu